{
  "gene_symbol": "GABRA4",
  "gene_name": "Gamma-aminobutyric acid receptor subunit alpha-4",
  "gene": "UniProtKB:P48169",
  "term_id": "GO:0007214",
  "term_label": "gamma-aminobutyric acid signaling pathway"
}